{
  "term_label": "Unknown molecular function",
  "gene_name": "Chondrosarcoma-associated gene 1 protein",
  "gene": "UniProtKB:Q6PB30",
  "gene_symbol": "CSAG1",
  "term_id": "UNKNOWN:0001"
}